nucleoside monophosphate catabolic process [GO:0009125] (biological process) Definition: The chemical reactions and pathways resulting in the breakdown of a nucleoside monophosphate, a compound consisting of a nucleobase linked to a deoxyribose or ribose sugar esterified with phosphate on the sugar. Also known as: nucleoside monophosphate breakdown, nucleoside monophosphate catabolism, nucleoside monophosphate degradation Relationships: is a type of GO:0009123; is a type of nucleoside phosphate catabolic process [GO:1901292] Subtypes: purine nucleoside monophosphate catabolic process [GO:0009128], pyrimidine nucleoside monophosphate catabolic process [GO:0009131], ribonucleoside monophosphate catabolic process [GO:0009158], deoxyribonucleoside monophosphate catabolic process [GO:0009159] Sources: GOC:go_curators, ISBN:0198506732